enterobacterial common antigen biosynthetic process [GO:0009246] (biological process) Relationships: is_a polysaccharide biosynthetic process [GO:0000271]; is a type of enterobacterial common antigen metabolic process [GO:0046378]; is a type of carbohydrate derivative biosynthetic process [GO:1901137] Sources: GOC:ma Definition: The chemical reactions and pathways resulting in the formation of the enterobacterial common antigen, an acidic polysaccharide containing N-acetyl-D-glucosamine, N-acetyl-D-mannosaminouronic acid, and 4-acetamido-4,6-dideoxy-D-galactose. A major component of the cell wall outer membrane of Gram-negative bacteria. Also known as: enterobacterial common antigen anabolism, enterobacterial common antigen biosynthesis, enterobacterial common antigen formation, enterobacterial common antigen synthesis